positive regulation of protein O-linked glycosylation [GO:1904100] (biological process) Relationships: is a type of positive regulation of glycoprotein biosynthetic process [GO:0010560]; is a type of regulation of protein O-linked glycosylation [GO:1904098]; positively regulates protein O-linked glycosylation [GO:0006493] Also known as: positive regulation of protein amino acid O-linked glycosylation, up regulation of protein O-linked glycosylation, up regulation of protein amino acid O-linked glycosylation, up-regulation of protein O-linked glycosylation, up-regulation of protein amino acid O-linked glycosylation, upregulation of protein O-linked glycosylation, upregulation of protein amino acid O-linked glycosylation, activation of protein O-linked glycosylation, activation of protein amino acid O-linked glycosylation Definition: Any process that activates or increases the frequency, rate or extent of protein O-linked glycosylation. References: PMID:24509081 Sources: GOC:TermGenie, GO_REF:0000058 Subtypes: GO:0010909